IgD binding [GO:0043472] (molecular function) References: PMID:12886015 Definition: Binding to an immunoglobulin of a D isotype. Relationships: is a type of GO:0019865